{
  "gene": "UniProtKB:Q7Z6K3",
  "term_label": "cytoplasm",
  "term_id": "GO:0005737",
  "gene_name": "Protein prenyltransferase alpha subunit repeat-containing protein 1",
  "gene_symbol": "PTAR1"
}